salivary gland cavitation [GO:0060662] (biological process) Definition: The process in which the solid core of salivary epithelium gives rise to the hollow tube of the gland. Sources: GOC:dph Also known as: salivary gland invagination Relationships: is a type of tube lumen cavitation [GO:0060605]; is part of GO:0007435